{
  "gene_name": "Apelin receptor",
  "term_label": "apelin receptor activity",
  "gene": "UniProtKB:P35414",
  "gene_symbol": "APLNR",
  "term_id": "GO:0060182"
}